methylammonium channel activity [GO:0015264] (molecular function) Relationships: is a type of methylammonium transmembrane transporter activity [GO:0015200]; is a type of channel activity [GO:0015267] Sources: GOC:mtg_transport, GOC:pr Definition: Enables the energy-independent facilitated diffusion of methylammonium through a transmembrane aqueous pore or channel. Methylammonium is CH3NH2.